{
  "gene_name": "Serpin B5",
  "gene": "UniProtKB:P36952",
  "term_id": "GO:0005615",
  "term_label": "extracellular space",
  "gene_symbol": "SERPINB5"
}